{
  "term_id": "GO:0015908",
  "term_label": "fatty acid transport",
  "gene_symbol": "FABP6",
  "gene": "UniProtKB:P51161",
  "gene_name": "Gastrotropin"
}